lamin binding [GO:0005521] (molecular function) Definition: Binding to lamin; any of a group of intermediate-filament proteins that form the fibrous matrix on the inner surface of the nuclear envelope. Relationships: is a type of GO:0005515 Sources: GOC:jl, ISBN:0198506732 Also known as: lamin/chromatin binding